U12-type post-spliceosomal complex [GO:0071022] (cellular component) Sources: GOC:krc, GOC:mah, ISBN:0879695897, ISBN:0879697393 Relationships: is a type of U12-type spliceosomal complex [GO:0005689]; is a type of post-spliceosomal complex [GO:0071020]; has part U6atac snRNP [GO:0005691]; has part U12 snRNP [GO:0005693] Definition: A spliceosomal complex that is formed following the second splicing event and contains the spliced product, the excised intron, and three snRNPs, U5, U12 and U6atac. Also known as: minor post-spliceosomal complex, AT-AC post-spliceosomal complex, mammalian U12-type spliceosomal complex C2, yeast U12-type spliceosomal complex A2-3